{
  "gene": "UniProtKB:P67812",
  "gene_name": "Signal peptidase complex catalytic subunit SEC11A",
  "gene_symbol": "SEC11A",
  "term_id": "GO:0006465",
  "term_label": "signal peptide processing"
}